{
  "gene_symbol": "CCNH",
  "term_label": "transcription initiation at RNA polymerase II promoter",
  "term_id": "GO:0006367",
  "gene": "UniProtKB:P51946",
  "gene_name": "Cyclin-H"
}